{
  "gene_name": "DENN domain-containing protein 1A",
  "term_id": "GO:0032456",
  "term_label": "endocytic recycling",
  "gene_symbol": "DENND1A",
  "gene": "UniProtKB:Q8TEH3"
}